{
  "term_id": "GO:0000122",
  "gene_name": "Transcription factor SOX-11",
  "term_label": "negative regulation of transcription by RNA polymerase II",
  "gene_symbol": "SOX11",
  "gene": "UniProtKB:P35716"
}